{
  "term_label": "protein sumoylation",
  "gene_symbol": "SUMO4",
  "term_id": "GO:0016925",
  "gene_name": "Small ubiquitin-related modifier 4",
  "gene": "UniProtKB:Q6EEV6"
}